positive regulation of catalytic activity [GO:0043085] (biological process) Relationships: is_a positive regulation of molecular function [GO:0044093]; is a type of GO:0050790; positively regulates GO:0003824 Definition: Any process that activates or increases the activity of an enzyme. Sources: GOC:ebc, GOC:jl, GOC:tb, GOC:vw Subtypes: positive regulation of cyclase activity [GO:0031281], positive regulation of deoxyribonuclease activity [GO:0032077], positive regulation of kinase activity [GO:0033674], positive regulation of helicase activity [GO:0051096], positive regulation of hydrolase activity [GO:0051345], positive regulation of lyase activity [GO:0051349], positive regulation of ligase activity [GO:0051351], positive regulation of oxidoreductase activity [GO:0051353], positive regulation of ubiquitin-protein transferase activity [GO:0051443], GO:0090045, positive regulation of protein-glutamine gamma-glutamyltransferase activity [GO:0150074], positive regulation of DNA-directed DNA polymerase activity [GO:1900264], positive regulation of serine C-palmitoyltransferase activity [GO:1904222], positive regulation of polynucleotide adenylyltransferase activity [GO:1904247], positive regulation of DNA topoisomerase (ATP-hydrolyzing) activity [GO:2000373], positive regulation of glycogen (starch) synthase activity [GO:2000467] Also known as: positive regulation of enzyme activity, up regulation of enzyme activity, up-regulation of enzyme activity, upregulation of enzyme activity, activation of enzyme activity, activation of metalloenzyme activity, positive regulation of metalloenzyme activity, stimulation of enzyme activity, stimulation of metalloenzyme activity, up regulation of metalloenzyme activity, up-regulation of metalloenzyme activity, upregulation of metalloenzyme activity